nuclear proteasome regulatory particle, base subcomplex [GO:0031610] (cellular component) Sources: GOC:mah Relationships: is a type of proteasome regulatory particle, base subcomplex [GO:0008540]; is a type of GO:0140513; is part of nuclear proteasome regulatory particle [GO:0031598] Definition: The subunits of the regulatory particle that directly associate with the core complex of a proteasome located in the nucleus of a cell.